{
  "gene": "UniProtKB:Q8NGC2",
  "gene_symbol": "OR4E2",
  "gene_name": "Olfactory receptor 4E2",
  "term_id": "GO:0005549",
  "term_label": "odorant binding"
}